{
  "term_label": "histone deacetylase activity",
  "gene": "UniProtKB:Q9UQL6",
  "gene_name": "Histone deacetylase 5",
  "term_id": "GO:0004407",
  "gene_symbol": "HDAC5"
}